positive regulation of meiotic nuclear division [GO:0045836] (biological process) Definition: Any process that activates or increases the frequency, rate or extent of meiosis. Sources: GOC:go_curators Also known as: positive regulation of meiosis, up regulation of meiosis, up-regulation of meiosis, upregulation of meiosis, activation of meiosis, stimulation of meiosis Relationships: is a type of regulation of meiotic nuclear division [GO:0040020]; is a type of positive regulation of meiotic cell cycle [GO:0051446]; is a type of positive regulation of nuclear division [GO:0051785]; is a type of positive regulation of cell cycle process [GO:0090068]; positively regulates meiotic nuclear division [GO:0140013] Subtypes: positive regulation of reciprocal meiotic recombination [GO:0010845], GO:0060903, activation of meiosis [GO:0090427]